protein localization to microtubule end [GO:1905725] (biological process) References: PMID:12034771 Sources: GOC:TermGenie, GO_REF:0000087 Definition: A process in which a protein is transported to, or maintained in, a location at a microtubule end. Relationships: is a type of protein localization to microtubule [GO:0035372] Also known as: protein localisation to microtubule end Subtypes: protein localization to microtubule minus-end [GO:1904519], protein localization to microtubule plus-end [GO:1904825]